{
  "term_label": "axon",
  "gene": "UniProtKB:P42858",
  "term_id": "GO:0030424",
  "gene_name": "Huntingtin",
  "gene_symbol": "HTT"
}